{
  "gene_name": "Prolactin-releasing peptide receptor",
  "term_label": "neuron projection",
  "gene_symbol": "PRLHR",
  "gene": "UniProtKB:P49683",
  "term_id": "GO:0043005"
}